ventral disc supernumerary microtubule array [GO:0097596] (cellular component) Note: Due to the asymmetric nature of the Giardia trophozoite, this term is defined spatially as the trophozoite is viewed from the dorsal side, with the two nuclei dorsal to the ventral disc, and the ventral disc toward the anterior. Relationships: is a type of cellular anatomical structure [GO:0110165]; is part of ventral disc [GO:0097597]; has part GO:0005874 Definition: A partial left-handed spiral array of microtubules that lies generally dorsal to the main ventral disc microtubule array in Giardia species (trophozoite stage). Also known as: supernumerary microtubule array, ventral disk supernumerary microtubule array Sources: GOC:giardia, ISBN:9780124260207